{
  "term_label": "Unknown biological process",
  "term_id": "UNKNOWN:0002",
  "gene": "UniProtKB:Q96PE3",
  "gene_name": "Inositol polyphosphate-4-phosphatase type I A",
  "gene_symbol": "INPP4A"
}